{
  "gene_symbol": "DAB2IP",
  "term_label": "Unknown cellular component",
  "gene": "UniProtKB:Q5VWQ8",
  "term_id": "UNKNOWN:0003",
  "gene_name": "Disabled homolog 2-interacting protein"
}